{
  "term_id": "UNKNOWN:0002",
  "gene": "UniProtKB:Q13287",
  "gene_name": "N-myc-interactor",
  "gene_symbol": "NMI",
  "term_label": "Unknown biological process"
}